{
  "term_id": "GO:0070776",
  "term_label": "MOZ/MORF histone acetyltransferase complex",
  "gene": "UniProtKB:Q8WYB5",
  "gene_name": "Histone acetyltransferase KAT6B",
  "gene_symbol": "KAT6B"
}